{
  "term_label": "calcium ion import across plasma membrane",
  "gene": "UniProtKB:O43497",
  "gene_symbol": "CACNA1G",
  "term_id": "GO:0098703",
  "gene_name": "Voltage-dependent T-type calcium channel subunit alpha-1G"
}